SLIK (SAGA-like) complex [GO:0046695] (cellular component) Definition: A SAGA-type histone acetyltransferase complex that contains a smaller form of Spt7 (lacking the SPT8 binding region) than the fungal SAGA complex, and consequently lacks Spt8. The complex is involved in the yeast retrograde response pathway, which is important for gene expression changes during mitochondrial dysfunction. References: PMID:33864814 Also known as: SAGA (alt) complex, SALSA complex, SLIK/SALSA complex Note: See also the cellular component term 'SAGA complex ; GO:0000124'. Relationships: is a type of SAGA-type complex [GO:0070461]; has part DUBm complex [GO:0071819]